{
  "gene_symbol": "ERMAP",
  "gene": "UniProtKB:Q96PL5",
  "gene_name": "Erythroid membrane-associated protein",
  "term_label": "external side of plasma membrane",
  "term_id": "GO:0009897"
}